{
  "term_id": "GO:0005886",
  "gene_name": "T cell receptor beta variable 6-1",
  "gene_symbol": "TRBV6-1",
  "term_label": "plasma membrane",
  "gene": "UniProtKB:A0A0K0K1D8"
}